labial disc morphogenesis [GO:0007454] (biological process) Definition: The process in which the anatomical structures derived from the labial disc are generated and organized. This includes the transformation of a labial imaginal disc from a monolayered epithelium in the larvae of holometabolous insects into recognizable adult structures including parts of the proboscis. Relationships: is a type of imaginal disc morphogenesis [GO:0007560]; is part of labial disc development [GO:0035217] Sources: GOC:bf, ISBN:0879694238 Also known as: labial disc metamorphosis